{
  "gene": "UniProtKB:O14669",
  "term_label": "blood coagulation",
  "gene_name": "Transmembrane gamma-carboxyglutamic acid protein 2",
  "gene_symbol": "PRRG2",
  "term_id": "GO:0007596"
}